{
  "term_id": "GO:1990349",
  "gene_symbol": "GJA8",
  "gene": "UniProtKB:P48165",
  "term_label": "gap junction-mediated intercellular transport",
  "gene_name": "Gap junction alpha-8 protein"
}